{
  "gene_name": "Syntaxin-binding protein 5-like",
  "term_label": "exocytosis",
  "gene_symbol": "STXBP5L",
  "gene": "UniProtKB:Q9Y2K9",
  "term_id": "GO:0006887"
}